low-affinity tryptophan transmembrane transporter activity [GO:0022893] (molecular function) Also known as: low-affinity tryptophan permease activity Sources: GOC:mtg_transport, ISBN:0815340729 Definition: Catalysis of the low-affinity transfer of L-tryptophan from one side of a membrane to the other. Tryptophan is 2-amino-3-(1H-indol-3-yl)propanoic acid. In low-affinity transport the transporter is able to bind the solute only if it is present at very high concentrations. Relationships: is a type of GO:0015196